{
  "term_label": "negative regulation of transcription by RNA polymerase II",
  "gene_symbol": "HEYL",
  "gene": "UniProtKB:Q9NQ87",
  "term_id": "GO:0000122",
  "gene_name": "Hairy_enhancer-of-split related with YRPW motif-like protein"
}